{
  "term_label": "regulation of transcription by RNA polymerase II",
  "gene_name": "Pancreas_duodenum homeobox protein 1",
  "gene_symbol": "PDX1",
  "gene": "UniProtKB:P52945",
  "term_id": "GO:0006357"
}